{
  "gene_symbol": "BID",
  "term_id": "GO:0008637",
  "gene": "UniProtKB:P55957",
  "term_label": "apoptotic mitochondrial changes",
  "gene_name": "BH3-interacting domain death agonist"
}